{
  "gene_name": "Neurexin-1",
  "term_id": "GO:0004888",
  "gene_symbol": "NRXN1",
  "term_label": "transmembrane signaling receptor activity",
  "gene": "UniProtKB:Q9ULB1"
}